{
  "gene": "UniProtKB:Q2TBC4",
  "term_label": "muscle alpha-actinin binding",
  "gene_name": "Prickle-like protein 4",
  "gene_symbol": "PRICKLE4",
  "term_id": "GO:0051371"
}